{
  "term_id": "UNKNOWN:0001",
  "gene_symbol": "C1orf53",
  "term_label": "Unknown molecular function",
  "gene": "UniProtKB:Q5VUE5",
  "gene_name": "Uncharacterized protein C1orf53"
}